{
  "term_id": "GO:0048489",
  "gene": "UniProtKB:O60282",
  "term_label": "synaptic vesicle transport",
  "gene_name": "Kinesin heavy chain isoform 5C",
  "gene_symbol": "KIF5C"
}